{
  "gene_symbol": "TMEFF1",
  "gene": "UniProtKB:Q8IYR6",
  "term_label": "host-mediated suppression of symbiont invasion",
  "term_id": "GO:0046597",
  "gene_name": "Tomoregulin-1"
}